{
  "term_label": "RNA polymerase II cis-regulatory region sequence-specific DNA binding",
  "term_id": "GO:0000978",
  "gene_symbol": "HOXA9",
  "gene": "UniProtKB:P31269",
  "gene_name": "Homeobox protein Hox-A9"
}